{
  "gene_name": "Cerebellin-3",
  "term_id": "GO:0043083",
  "gene_symbol": "CBLN3",
  "gene": "UniProtKB:Q6UW01",
  "term_label": "synaptic cleft"
}